negative regulation of ectoderm development [GO:2000384] (biological process) Definition: Any process that stops, prevents or reduces the frequency, rate or extent of ectoderm development. Sources: GOC:BHF Relationships: is a type of negative regulation of developmental process [GO:0051093]; is_a regulation of ectoderm development [GO:2000383]; negatively regulates GO:0007398